lipoprotein releasing activity [GO:0140306] (molecular function) References: PMID:10783239, PMID:21670534 Relationships: is_a protein transporter activity [GO:0140318] Definition: The activity of recognizing mature outer membrane lipoproteins in the inner membrane and releasing from the inner membrane so that they can be transported across the periplasmic space to their target location, the outer membrane. This function exists in diderm bacteria, mediated by the LolCDE complex.